{
  "term_id": "GO:0007010",
  "term_label": "cytoskeleton organization",
  "gene_name": "Microtubule-associated serine_threonine-protein kinase 3",
  "gene_symbol": "MAST3",
  "gene": "UniProtKB:O60307"
}